{
  "term_label": "intracellular potassium ion homeostasis",
  "gene": "UniProtKB:P05026",
  "gene_symbol": "ATP1B1",
  "term_id": "GO:0030007",
  "gene_name": "Sodium_potassium-transporting ATPase subunit beta-1"
}